{
  "term_label": "cadherin binding",
  "term_id": "GO:0045296",
  "gene_name": "Receptor-type tyrosine-protein phosphatase beta",
  "gene": "UniProtKB:P23467",
  "gene_symbol": "PTPRB"
}